{
  "gene_name": "Dixin",
  "term_id": "GO:0005829",
  "term_label": "cytosol",
  "gene": "UniProtKB:Q155Q3",
  "gene_symbol": "DIXDC1"
}